regulation of interleukin-7 production [GO:0032676] (biological process) Subtypes: negative regulation of interleukin-7 production [GO:0032716], positive regulation of interleukin-7 production [GO:0032756] Definition: Any process that modulates the frequency, rate, or extent of interleukin-7 production. Also known as: regulation of IL-7 production, regulation of interleukin-7 biosynthetic process, regulation of interleukin-7 secretion Relationships: is a type of GO:0001817; regulates interleukin-7 production [GO:0032636] References: PMID:25962782 Sources: GOC:mah